myosin filament organization [GO:0031033] (biological process) Note: Note that this term is a child of 'actin cytoskeleton organization and biogenesis ; GO:0030036' because the actin cytoskeleton is defined as actin filaments and associated proteins; myosin structures are sufficiently closely associated with actin filaments to be included with the actin cytoskeleton. Definition: A process that is carried out at the cellular level which results in the assembly, arrangement of constituent parts, or disassembly of a filament composed of myosin molecules. Also known as: myosin filament organisation, myosin filament assembly or disassembly, myosin polymerization or depolymerization Relationships: is a type of actin cytoskeleton organization [GO:0030036]; is_a GO:0097435 Subtypes: myosin filament assembly [GO:0031034], myosin filament disassembly [GO:0031035], myosin II filament organization [GO:0031038] Sources: GOC:mah